{
  "term_label": "mitotic G2 DNA damage checkpoint signaling",
  "term_id": "GO:0007095",
  "gene_name": "BRISC and BRCA1-A complex member 1",
  "gene": "UniProtKB:Q9NWV8",
  "gene_symbol": "BABAM1"
}